inositol 3-alpha-galactosyltransferase activity [GO:0047216] (molecular function) Relationships: is a type of UDP-galactosyltransferase activity [GO:0035250] Definition: Catalysis of the reaction: myo-inositol + UDP-galactose = O-alpha-D-galactosyl-(1,3)-1D-myo-inositol + UDP. Also known as: inositol 1-alpha-galactosyltransferase activity, UDP-D-galactose:inositol galactosyltransferase activity, UDP-galactose:myo-inositol 1-alpha-D-galactosyltransferase activity, UDP-galactose:myo-inositol 3-alpha-D-galactosyltransferase activity, UDPgalactose:myo-inositol 1-alpha-D-galactosyltransferase activity, galactinol synthase activity, uridine diphosphogalactose-inositol galactosyltransferase activity Sources: EC:2.4.1.123, MetaCyc:2.4.1.123-RXN